metanephric podocyte differentiation [GO:0072248] (biological process) Also known as: metanephric glomerular visceral epithelial cell differentiation Sources: GOC:mtg_kidney_jan10 Relationships: is a type of GO:0072112; is a type of GO:0072312 Definition: The process in which a relatively unspecialized cell acquires specialized features of a metanephric glomerular visceral epithelial cell. A metanephric glomerular visceral epithelial cell is a specialized epithelial cell that contains 'feet' that interdigitate with the 'feet' of other glomerular epithelial cells in the metanephros.